anesthesia-resistant memory [GO:0007615] (biological process) Definition: The memory process that results in the formation of consolidated memory resistant to disruption of the patterned activity of the brain, without requiring protein synthesis. References: PMID:15143285, PMID:17088531 Relationships: is_a memory [GO:0007613]